{
  "term_id": "GO:0097500",
  "gene": "UniProtKB:Q5H913",
  "term_label": "receptor localization to non-motile cilium",
  "gene_name": "ADP-ribosylation factor-like protein 13A",
  "gene_symbol": "ARL13A"
}